{
  "gene_symbol": "PRAMEF27",
  "term_label": "cytoplasm",
  "gene": "UniProtKB:A3QJZ7",
  "term_id": "GO:0005737",
  "gene_name": "PRAME family member 27"
}